{
  "term_label": "nucleus",
  "term_id": "GO:0005634",
  "gene": "UniProtKB:A5LHX3",
  "gene_symbol": "PSMB11",
  "gene_name": "Proteasome subunit beta type-11"
}